{
  "gene": "UniProtKB:P01857",
  "gene_symbol": "IGHG1",
  "term_id": "GO:0042571",
  "term_label": "immunoglobulin complex, circulating",
  "gene_name": "Immunoglobulin heavy constant gamma 1"
}